{
  "gene_symbol": "GRIN2B",
  "gene": "UniProtKB:Q13224",
  "term_id": "GO:0035249",
  "gene_name": "Glutamate receptor ionotropic, NMDA 2B",
  "term_label": "synaptic transmission, glutamatergic"
}